regulation of branching involved in ureteric bud morphogenesis [GO:0090189] (biological process) Subtypes: positive regulation of branching involved in ureteric bud morphogenesis [GO:0090190], negative regulation of branching involved in ureteric bud morphogenesis [GO:0090191] Sources: GOC:dph, GOC:tb, GOC:yaf Definition: Any process that modulates the rate, frequency or extent of branching involved in ureteric bud morphogenesis, the process in which the branching structure of the ureteric bud is generated and organized. The ureteric bud is an epithelial tube that grows out from the metanephric duct. The bud elongates and branches to give rise to the ureter and kidney collecting tubules. Relationships: is_a regulation of morphogenesis of a branching structure [GO:0060688]; is a type of regulation of kidney development [GO:0090183]; is a type of regulation of morphogenesis of an epithelium [GO:1905330]; is a type of regulation of animal organ morphogenesis [GO:2000027]; regulates GO:0001658